aldoxime metabolic process [GO:0019330] (biological process) Subtypes: GO:0046307, Z-phenylacetaldoxime catabolic process [GO:0046308] Also known as: aldoxime metabolism Sources: GOC:curators Definition: The chemical reactions and pathways involving aldoximes, compounds derived by the reaction of an aldose with hydroxylamine, thus containing the aldoxime group -HC=NOH. Relationships: is a type of metabolic process [GO:0008152]